copper ion transmembrane transport [GO:0035434] (biological process) Note: Note that this term is not intended for use in annotating lateral movement within membranes. Regulation: regulated by regulation of copper ion transmembrane transport [GO:1902311]; negatively regulated by GO:1902312; positively regulated by positive regulation of copper ion transmembrane transport [GO:1902313] Also known as: copper cation transmembrane transport, copper ion membrane transport Subtypes: GO:0015679, copper ion export [GO:0060003], copper ion import across prospore membrane [GO:0097430], GO:0140145, copper import into the mitochondrion [GO:0140636] Relationships: is a type of copper ion transport [GO:0006825]; is_a monoatomic cation transmembrane transport [GO:0098655] Definition: The directed movement of copper cation across a membrane. Sources: GOC:vw